{
  "term_label": "tRNA wobble uridine modification",
  "term_id": "GO:0002098",
  "gene_name": "Probable tRNA methyltransferase 9B",
  "gene_symbol": "TRMT9B",
  "gene": "UniProtKB:Q9P272"
}